{
  "term_label": "plasma membrane",
  "gene": "UniProtKB:P22607",
  "term_id": "GO:0005886",
  "gene_symbol": "FGFR3",
  "gene_name": "Fibroblast growth factor receptor 3"
}